{
  "term_id": "GO:0005886",
  "term_label": "plasma membrane",
  "gene_name": "Killer cell immunoglobulin-like receptor 2DL5A",
  "gene": "UniProtKB:Q8N109",
  "gene_symbol": "KIR2DL5A"
}